{
  "term_id": "UNKNOWN:0003",
  "gene_name": "Pleckstrin homology domain-containing family M member 1",
  "gene_symbol": "PLEKHM1",
  "term_label": "Unknown cellular component",
  "gene": "UniProtKB:Q9Y4G2"
}